phosphoribosylaminoimidazole carboxylase complex [GO:0009320] (cellular component) Relationships: is a type of catalytic complex [GO:1902494]; BFO_0000050 GO:0005737 Definition: A protein complex that possesses phosphoribosylaminoimidazole carboxylase activity. Sources: GOC:mah Note: See also the molecular function term 'phosphoribosylaminoimidazole carboxylase activity ; GO:0004638'.